specification of axis polarity [GO:0065001] (biological process) Relationships: is a type of pattern specification process [GO:0007389]; is part of axis specification [GO:0009798] Definition: The pattern specification process in which the polarity of a body or organ axis is established and maintained. Subtypes: polarity specification of adaxial/abaxial axis [GO:0009944], GO:0009949, polarity specification of dorsal/ventral axis [GO:0009951], GO:0010084, polarity specification of proximal/distal axis [GO:0010085], specification of plant organ axis polarity [GO:0090708] Sources: GOC:mah